{
  "gene_symbol": "ORAI1",
  "gene_name": "Calcium release-activated calcium channel protein 1",
  "term_id": "GO:0015279",
  "gene": "UniProtKB:Q96D31",
  "term_label": "store-operated calcium channel activity"
}